{
  "term_id": "GO:0003755",
  "gene_name": "Peptidyl-prolyl cis-trans isomerase A-like 4F",
  "gene": "UniProtKB:P0DN26",
  "gene_symbol": "PPIAL4F",
  "term_label": "peptidyl-prolyl cis-trans isomerase activity"
}